{
  "term_id": "GO:0038184",
  "gene": "UniProtKB:Q8TDU6",
  "term_label": "adenylate cyclase-activating G protein-coupled bile acid receptor signaling pathway",
  "gene_name": "G-protein coupled bile acid receptor 1",
  "gene_symbol": "GPBAR1"
}